{
  "gene_name": "Nutritionally-regulated adipose and cardiac enriched protein homolog",
  "gene": "UniProtKB:Q8N912",
  "term_id": "GO:0005886",
  "term_label": "plasma membrane",
  "gene_symbol": "NRAC"
}